{
  "term_label": "transcription corepressor activity",
  "gene_symbol": "PARP9",
  "gene": "UniProtKB:Q8IXQ6",
  "term_id": "GO:0003714",
  "gene_name": "Protein mono-ADP-ribosyltransferase PARP9"
}